{
  "gene_name": "1-phosphatidylinositol 4,5-bisphosphate phosphodiesterase beta-1",
  "term_label": "phosphatidylinositol metabolic process",
  "term_id": "GO:0046488",
  "gene_symbol": "PLCB1",
  "gene": "UniProtKB:Q9NQ66"
}